{
  "gene": "UniProtKB:Q96EX3",
  "gene_name": "Cytoplasmic dynein 2 intermediate chain 2",
  "term_id": "GO:0097014",
  "term_label": "ciliary plasm",
  "gene_symbol": "DYNC2I2"
}